{
  "term_label": "Unknown molecular function",
  "gene_name": "Putative uncharacterized protein encoded by LINC00269",
  "gene_symbol": "LINC00269",
  "gene": "UniProtKB:Q8N2A0",
  "term_id": "UNKNOWN:0001"
}